endoplasmic reticulum membrane [GO:0005789] (cellular component) Relationships: is a type of organelle membrane [GO:0031090]; is part of nuclear outer membrane-endoplasmic reticulum membrane network [GO:0042175]; is part of endoplasmic reticulum subcompartment [GO:0098827] Subtypes: rough endoplasmic reticulum membrane [GO:0030867], smooth endoplasmic reticulum membrane [GO:0030868], sarcoplasmic reticulum membrane [GO:0033017], endoplasmic reticulum tubular network membrane [GO:0098826] Definition: The lipid bilayer surrounding the endoplasmic reticulum. Also known as: ER membrane Sources: GOC:mah